neuron projection extension involved in neuron projection guidance [GO:1902284] (biological process) Definition: Any neuron projection extension that is involved in neuron projection guidance. Also known as: neuron process extension involved in neuron process guidance, neuron process extension involved in neuron projection guidance, neuron process extension involved in neuron protrusion guidance, neuron process extension involved in neuronal cell projection guidance, neuron projection extension involved in neuron process guidance, neuron projection extension involved in neuron protrusion guidance, neuron projection extension involved in neuronal cell projection guidance, neuron protrusion extension involved in neuron process guidance, neuron protrusion extension involved in neuron projection guidance, neuron protrusion extension involved in neuron protrusion guidance, neuron protrusion extension involved in neuronal cell projection guidance, neuronal cell projection extension involved in neuron process guidance, neuronal cell projection extension involved in neuron projection guidance, neuronal cell projection extension involved in neuron protrusion guidance, neuronal cell projection extension involved in neuronal cell projection guidance, neurite extension involved in neurite guidance, neurite extension involved in neuron process guidance, neurite extension involved in neuron projection guidance, neurite extension involved in neuron protrusion guidance, neurite extension involved in neuronal cell projection guidance, neuron process extension involved in neurite guidance, neuron projection extension involved in neurite guidance, neuron protrusion extension involved in neurite guidance, neuronal cell projection extension involved in neurite guidance References: PMID:22790009 Sources: GOC:BHF, GOC:TermGenie, GOC:rl Relationships: is a type of neuron projection extension [GO:1990138]; is part of neuron projection guidance [GO:0097485] Subtypes: GO:0048846